epithelial cell migration involved in metanephric proximal tubule morphogenesis [GO:0072292] (biological process) Relationships: is a type of GO:0072159; is a type of epithelial cell migration involved in metanephric nephron tubule morphogenesis [GO:0072290]; is part of metanephric proximal tubule morphogenesis [GO:0072288] Sources: GOC:mtg_kidney_jan10 Definition: The orderly movement of epithelial cells within a renal tubule that contributes to metanephric proximal tubule morphogenesis.